dorsal closure, spreading of leading edge cells [GO:0007395] (biological process) Definition: Dorsally-directed movement of a cell at the leading edge of the epithelium over the amnioserosa. References: PMID:12147138 Sources: GOC:bf Relationships: is_a GO:0016477; is part of GO:0007391